{
  "gene_name": "Glycerol kinase 3",
  "term_label": "glycerol metabolic process",
  "term_id": "GO:0006071",
  "gene_symbol": "GK3",
  "gene": "UniProtKB:Q14409"
}